{
  "term_id": "UNKNOWN:0003",
  "gene_name": "Lymphocyte expansion molecule",
  "gene": "UniProtKB:Q3ZCV2",
  "gene_symbol": "LEXM",
  "term_label": "Unknown cellular component"
}